{
  "gene_name": "Ras-related protein Rab-28",
  "gene_symbol": "RAB28",
  "term_label": "endomembrane system",
  "gene": "UniProtKB:P51157",
  "term_id": "GO:0012505"
}